beta-D-galactosyl-(1->3)-N-acetyl-beta-D-galactosaminide alpha-2,3- sialyltransferase [GO:0047288] (molecular function) Relationships: is a type of GO:0008373 Definition: Catalysis of the reaction: beta-D-galactosyl-(1->3)-N-acetyl-beta-D-galactosaminyl derivative + CMP-N-acetyl-beta-neuraminate = N-acetyl-alpha-neuraminyl-(2->3)-beta-D-galactosyl-(1->3)-N-acetyl-beta-D-galactosaminyl derivative + CMP + H+. Sources: EC:2.4.3.2, MetaCyc:2.4.99.2-RXN Also known as: monosialoganglioside sialyltransferase